{
  "term_label": "phospholipid dephosphorylation",
  "gene": "UniProtKB:O14495",
  "term_id": "GO:0046839",
  "gene_symbol": "PLPP3",
  "gene_name": "Phospholipid phosphatase 3"
}